{
  "gene_symbol": "CFD",
  "term_id": "GO:0051604",
  "term_label": "protein maturation",
  "gene_name": "Complement factor D",
  "gene": "UniProtKB:P00746"
}